amylopectin metabolic process [GO:2000896] (biological process) Sources: GOC:mengo_curators Subtypes: GO:0010021, amylopectin catabolic process [GO:2000897] Definition: The chemical reactions and pathways involving an amylopectin. Also known as: Amylopectin metabolism Relationships: is a type of macromolecule metabolic process [GO:0043170]; is a type of carbohydrate derivative metabolic process [GO:1901135]